platelet-derived growth factor complex [GO:1990265] (cellular component) Relationships: is a type of growth factor complex [GO:0036454] Definition: A protein complex consisting of two chains of platelet-derived growth factor (PDGF) subunits. PDGF dimers bind to PDGF receptors in the plasma membrane and induce receptor dimerization and activation. PDGFs are involved in a wide variety of signaling processes. PDGFs are found in all vertebrates where at least 2 different chains (A and B) exist. In human (and other mammals), four types of PDGF chains (A, B, C, and D) are known which form five different dimers (AA, AB, BB, CC and DD). References: PMID:11331882 Sources: GOC:bhm Note: An example of this is PDGFA in human (P04085) in PMID:20534510 (inferred from direct assay). Also known as: PDGF-AA dimer, PDGF-AB dimer, PDGF-BB dimer, PDGF-CC dimer, PDGF-DD dimer, PDGF complex